{
  "term_label": "nucleosome",
  "gene_name": "Spermatid nuclear transition protein 1",
  "gene": "UniProtKB:P09430",
  "gene_symbol": "TNP1",
  "term_id": "GO:0000786"
}